{
  "gene": "UniProtKB:Q9HBF5",
  "gene_name": "Suppressor of tumorigenicity 20 protein",
  "term_label": "Unknown biological process",
  "gene_symbol": "ST20",
  "term_id": "UNKNOWN:0002"
}